{
  "gene": "UniProtKB:Q9BY11",
  "gene_name": "Protein kinase C and casein kinase substrate in neurons protein 1",
  "gene_symbol": "PACSIN1",
  "term_label": "regulation of endocytosis",
  "term_id": "GO:0030100"
}